{
  "gene_name": "Podocalyxin",
  "term_label": "microvillus membrane",
  "gene": "UniProtKB:O00592",
  "term_id": "GO:0031528",
  "gene_symbol": "PODXL"
}